{
  "term_label": "heme binding",
  "gene": "UniProtKB:Q6B0K9",
  "gene_symbol": "HBM",
  "term_id": "GO:0020037",
  "gene_name": "Hemoglobin subunit mu"
}